{
  "gene_symbol": "KDM4C",
  "term_label": "chromatin remodeling",
  "term_id": "GO:0006338",
  "gene_name": "Lysine-specific demethylase 4C",
  "gene": "UniProtKB:Q9H3R0"
}